antigen processing and presentation of peptide antigen via MHC class II [GO:0002495] (biological process) References: PMID:15531770, PMID:15771591 Sources: GOC:add, ISBN:0781735149 Definition: The process in which an antigen-presenting cell expresses a peptide antigen on its cell surface in association with an MHC class II protein complex. The peptide antigen is typically, but not always, processed from a whole protein. Subtypes: GO:0002491, antigen processing and presentation of exogenous peptide antigen via MHC class II [GO:0019886] Relationships: is a type of antigen processing and presentation of peptide or polysaccharide antigen via MHC class II [GO:0002504]; is a type of GO:0048002 Also known as: peptide antigen processing and presentation via MHC class II Regulation: regulated by regulation of antigen processing and presentation of peptide antigen via MHC class II [GO:0002586]; negatively regulated by GO:0002587; positively regulated by positive regulation of antigen processing and presentation of peptide antigen via MHC class II [GO:0002588]